{
  "gene": "UniProtKB:Q9NPI9",
  "term_label": "plasma membrane",
  "term_id": "GO:0005886",
  "gene_symbol": "KCNJ16",
  "gene_name": "Inward rectifier potassium channel 16"
}